{
  "term_id": "GO:0051289",
  "gene_symbol": "GNMT",
  "gene": "UniProtKB:Q14749",
  "term_label": "protein homotetramerization",
  "gene_name": "Glycine N-methyltransferase"
}